{
  "gene_symbol": "CCR1",
  "gene_name": "C-C chemokine receptor type 1",
  "gene": "UniProtKB:P32246",
  "term_id": "GO:0005737",
  "term_label": "cytoplasm"
}